positive regulation of mediator complex assembly [GO:2001178] (biological process) Definition: Any process that activates or increases the frequency, rate or extent of mediator complex assembly. Relationships: is a type of positive regulation of protein-containing complex assembly [GO:0031334]; is a type of GO:2001176; positively regulates mediator complex assembly [GO:0036034] Sources: GOC:obol